{
  "gene": "UniProtKB:Q9H4I2",
  "gene_symbol": "ZHX3",
  "term_id": "GO:0000981",
  "gene_name": "Zinc fingers and homeoboxes protein 3",
  "term_label": "DNA-binding transcription factor activity, RNA polymerase II-specific"
}